positive regulation of dorsal/ventral axon guidance [GO:1905817] (biological process) Definition: Any process that activates or increases the frequency, rate or extent of dorsal/ventral axon guidance. Relationships: is a type of positive regulation of axon guidance [GO:1902669]; is a type of GO:1905815; positively regulates dorsal/ventral axon guidance [GO:0033563] References: PMID:18434533 Sources: GOC:TermGenie, GO_REF:0000058 Also known as: positive regulation of dorsal-ventral axon guidance, positive regulation of dorsal/ventral axon pathfinding, positive regulation of dorsoventral axon guidance, up regulation of dorsal-ventral axon guidance, up regulation of dorsal/ventral axon guidance, up regulation of dorsal/ventral axon pathfinding, up regulation of dorsoventral axon guidance, up-regulation of dorsal-ventral axon guidance, up-regulation of dorsal/ventral axon guidance, up-regulation of dorsal/ventral axon pathfinding, up-regulation of dorsoventral axon guidance, upregulation of dorsal-ventral axon guidance, upregulation of dorsal/ventral axon guidance, upregulation of dorsal/ventral axon pathfinding, upregulation of dorsoventral axon guidance, activation of dorsal-ventral axon guidance, activation of dorsal/ventral axon guidance, activation of dorsal/ventral axon pathfinding, activation of dorsoventral axon guidance